negative regulation of fatty acid beta-oxidation [GO:0031999] (biological process) Subtypes: negative regulation of fatty acid beta-oxidation using acyl-CoA dehydrogenase [GO:1904736] Definition: Any process that stops, prevents, or reduces the frequency, rate or extent of fatty acid beta-oxidation. Relationships: is a type of regulation of fatty acid beta-oxidation [GO:0031998]; is a type of negative regulation of fatty acid oxidation [GO:0046322]; is_a GO:0050995; negatively regulates fatty acid beta-oxidation [GO:0006635] Also known as: down regulation of fatty acid beta-oxidation, down-regulation of fatty acid beta-oxidation, downregulation of fatty acid beta-oxidation, inhibition of fatty acid beta-oxidation Sources: GOC:mah